processes downstream of sex determination signal [GO:0007545] (biological process) Subtypes: somatic processes downstream of sex determination signal [GO:0007546], germ-line processes downstream of sex determination signal [GO:0007547] Sources: GOC:mah Definition: The sex determination processes that take place after the initial transmission of the sexual phenotype to specific information pathways. Relationships: is a type of sex determination [GO:0007530]; is part of multicellular organism development [GO:0007275]